{
  "term_id": "GO:0004197",
  "gene_symbol": "LGMN",
  "gene": "UniProtKB:Q99538",
  "gene_name": "Legumain",
  "term_label": "cysteine-type endopeptidase activity"
}